{
  "gene_name": "Transmembrane protein 275",
  "gene_symbol": "TMEM275",
  "gene": "UniProtKB:A0A0U1RQS6",
  "term_id": "UNKNOWN:0002",
  "term_label": "Unknown biological process"
}